N2-acetyl-L-ornithine:2-oxoglutarate 5-aminotransferase activity [GO:0003992] (molecular function) Sources: EC:2.6.1.11, RHEA:18049 Also known as: acetylornithine aminotransferase activity, acetylornithine transaminase activity, succinylornithine aminotransferase activity, N2-acetylornithine 5-aminotransferase activity, 2-N-acetyl-L-ornithine:2-oxoglutarate 5-aminotransferase activity, ACOAT activity, N(2)-acetylornithine 5-transaminase activity, N-acetylornithine aminotransferase activity, N-acetylornithine-delta-transaminase activity, N2-acetyl-L-ornithine:2-oxoglutarate aminotransferase activity, N2-acetylornithine 5-transaminase activity, acetylornithine 5-aminotransferase activity, acetylornithine delta-transaminase activity Relationships: is a type of GO:0008483 Definition: Catalysis of the reaction: 2-oxoglutarate + N(2)-acetyl-L-ornithine = N-acetyl-L-glutamate 5-semialdehyde + L-glutamate.